SHREC complex [GO:0070824] (cellular component) Also known as: Snf2/HDAC containing repressor complex, Snf2/Hdac repressive complex References: PMID:17289569 Sources: GOC:mah Relationships: is a type of NuRD complex [GO:0016581] Definition: A histone deacetylase complex that contains a core of four proteins -- Clr1, Clr2, Clr3, and Mit1 in fission yeast -- and localizes to all heterochromatic regions in the genome as well as some euchromatic sites. The complex is involved in regulating nucleosome positioning to assemble higher-order chromatin structures.